{
  "term_label": "growth cone",
  "term_id": "GO:0030426",
  "gene_symbol": "STMN2",
  "gene": "UniProtKB:Q93045",
  "gene_name": "Stathmin-2"
}